{
  "term_id": "GO:0017083",
  "gene_name": "4-galactosyl-N-acetylglucosaminide 3-alpha-L-fucosyltransferase FUT5",
  "term_label": "4-galactosyl-N-acetylglucosaminide 3-alpha-L-fucosyltransferase activity",
  "gene_symbol": "FUT5",
  "gene": "UniProtKB:Q11128"
}